{
  "gene": "UniProtKB:Q9Y6H3",
  "term_id": "UNKNOWN:0001",
  "term_label": "Unknown molecular function",
  "gene_symbol": "ATP23",
  "gene_name": "Mitochondrial inner membrane protease ATP23 homolog"
}